photoreceptor cell axon guidance [GO:0072499] (biological process) Definition: The chemotaxis process that directs the migration of a photoreceptor cell axon growth cone to its target in the optic lobe in response to a combination of attractive and repulsive cues. References: PMID:20826677 Sources: GOC:sart Also known as: photoreceptor cell axon pathfinding Relationships: is a type of axon guidance [GO:0007411] Regulation: RO_0002211 by regulation of photoreceptor cell axon guidance [GO:2000289]